{
  "gene_symbol": "CSNK2A1",
  "gene": "UniProtKB:P68400",
  "term_label": "protein kinase CK2 complex",
  "term_id": "GO:0005956",
  "gene_name": "Casein kinase II subunit alpha"
}